{
  "gene_name": "WD repeat-containing protein 49",
  "gene": "UniProtKB:Q8IV35",
  "gene_symbol": "WDR49",
  "term_label": "Unknown cellular component",
  "term_id": "UNKNOWN:0003"
}